{
  "term_label": "RNA polymerase II cis-regulatory region sequence-specific DNA binding",
  "gene_symbol": "POU2F2",
  "gene_name": "POU domain, class 2, transcription factor 2",
  "gene": "UniProtKB:P09086",
  "term_id": "GO:0000978"
}